{
  "gene": "UniProtKB:P49116",
  "gene_name": "Nuclear receptor subfamily 2 group C member 2",
  "term_id": "GO:0040019",
  "gene_symbol": "NR2C2",
  "term_label": "positive regulation of embryonic development"
}